{
  "gene": "UniProtKB:Q5IJ48",
  "term_id": "UNKNOWN:0001",
  "term_label": "Unknown molecular function",
  "gene_name": "Protein crumbs homolog 2",
  "gene_symbol": "CRB2"
}